gene conversion of immunoglobulin genes involved in immune response [GO:0002207] (biological process) Also known as: gene conversion of antibody genes during immune response, gene conversion of immunoglobulin genes during immune response Relationships: is_a gene conversion of immunoglobulin genes [GO:0002206]; is a type of somatic diversification of immunoglobulins involved in immune response [GO:0002208] Definition: The somatic process in which immunoglobulin genes are diversified through the mechanism of gene conversion following the induction of and contributing to an immune response. References: PMID:14991701 Sources: GOC:add